{
  "term_id": "GO:0001849",
  "gene_name": "Serum amyloid P-component",
  "gene": "UniProtKB:P02743",
  "gene_symbol": "APCS",
  "term_label": "complement component C1q complex binding"
}